negative regulation of systemic acquired resistance [GO:0010113] (biological process) Definition: Any process that stops, prevents, or reduces the frequency, rate or extent of systemic acquired resistance. Relationships: is_a negative regulation of response to biotic stimulus [GO:0002832]; is a type of regulation of systemic acquired resistance [GO:0010112]; is a type of negative regulation of defense response [GO:0031348]; is a type of negative regulation of response to external stimulus [GO:0032102]; negatively regulates systemic acquired resistance [GO:0009627] Sources: GOC:sm Also known as: down regulation of systemic acquired resistance, down-regulation of systemic acquired resistance, downregulation of systemic acquired resistance, inhibition of systemic acquired resistance